{
  "gene_name": "Putative transmembrane protein ENSP00000320207",
  "term_id": "UNKNOWN:0001",
  "term_label": "Unknown molecular function",
  "gene": "UniProtKB:A6NDX4",
  "gene_symbol": "A6NDX4"
}